extracellular matrix [GO:0031012] (CC) References: PMID:21123617, PMID:28089324, PMID:33605520 Sources: GOC:BHF, GOC:mah, GOC:rph Relationships: is a type of external encapsulating structure [GO:0030312] Also known as: proteinaceous extracellular matrix, matrisome Definition: A structure lying external to one or more cells, which provides structural support, biochemical or biomechanical cues for cells or tissues. Subtypes: basement membrane [GO:0005604], interstitial matrix [GO:0005614], specialized extracellular matrix [GO:0140047], basement membrane/interstitial matrix interface [GO:0140086]